{
  "term_id": "GO:0007188",
  "gene": "UniProtKB:A8MTJ3",
  "gene_symbol": "GNAT3",
  "term_label": "adenylate cyclase-modulating G protein-coupled receptor signaling pathway",
  "gene_name": "Guanine nucleotide-binding protein G(t) subunit alpha-3"
}